{
  "term_label": "neuron differentiation",
  "gene_symbol": "EGFR",
  "gene": "UniProtKB:P00533",
  "gene_name": "Epidermal growth factor receptor",
  "term_id": "GO:0030182"
}